{
  "gene_symbol": "H2BC12L",
  "gene": "UniProtKB:P57053",
  "term_label": "innate immune response in mucosa",
  "gene_name": "Histone H2B type F-S",
  "term_id": "GO:0002227"
}